{
  "term_id": "GO:0032095",
  "gene": "UniProtKB:Q9UBU3",
  "gene_symbol": "GHRL",
  "gene_name": "Appetite-regulating hormone",
  "term_label": "regulation of response to food"
}